{
  "gene": "UniProtKB:P08195",
  "term_id": "GO:0015823",
  "term_label": "phenylalanine transport",
  "gene_symbol": "SLC3A2",
  "gene_name": "4F2 cell-surface antigen heavy chain"
}